{
  "gene": "UniProtKB:P52952",
  "term_label": "nucleus",
  "gene_name": "Homeobox protein Nkx-2.5",
  "term_id": "GO:0005634",
  "gene_symbol": "NKX2-5"
}